mating projection base [GO:0001400] (cellular component) Also known as: base of shmoo tip, conjugation tube base Definition: The region where the mating projection meets the bulk of the cell, in unicellular fungi exposed to mating pheromone. Sources: GOC:mcc Relationships: is_a cellular anatomical structure [GO:0110165]; is part of mating projection [GO:0005937]